1-alpha,25-dihydroxyvitamin D3 23-hydroxylase activity [GO:0062181] (molecular function) References: PMID:22100522, PMID:30205156 Sources: RHEA:49192 Relationships: is a type of vitamin D 23-hydroxylase activity [GO:0062179] Definition: Catatlysis of the reaction: calcitriol + 2 H+ + O2 + 2 reduced [adrenodoxin] = 1alpha,23S,25-trihydroxycholecalciferol + H2O + 2 oxidized [adrenodoxin].